2-oxoglutarate-dependent tRNA 5-methylcytidine formyltransferase activity [GO:0160290] (molecular function) Relationships: is a type of 2-oxoglutarate-dependent dioxygenase activity [GO:0016706]; is a type of catalytic activity, acting on a tRNA [GO:0140101] Definition: Catalysis of the reaction: 5-methylcytidine(34) in mitochondrial tRNA(Met) + 2 2-oxoglutarate + 2 O2 = 5-formylcytidine(34) in mitochondrial tRNA(Met) + 2 succinate + 2 CO2 + H2O. References: PMID:27497299, PMID:28472312 Sources: RHEA:54144